{
  "term_label": "endosome",
  "gene": "UniProtKB:Q9UN37",
  "gene_name": "Vacuolar protein sorting-associated protein 4A",
  "gene_symbol": "VPS4A",
  "term_id": "GO:0005768"
}